Golgi lumen acidification [GO:0061795] (biological process) References: PMID:23447592 Sources: GOC:dph Relationships: is_a intracellular pH reduction [GO:0051452] Definition: Any process that reduces the pH of the Golgi lumen, measured by the concentration of the hydrogen ion. Regulation: regulated by regulation of Golgi lumen acidification [GO:1905526]; negatively regulated by negative regulation of Golgi lumen acidification [GO:1905527]; positively regulated by positive regulation of Golgi lumen acidification [GO:1905528] Also known as: Golgi apparatus lumen acidification